{
  "gene_name": "Glutamate-rich protein 6",
  "term_id": "UNKNOWN:0002",
  "gene_symbol": "ERICH6",
  "gene": "UniProtKB:Q7L0X2",
  "term_label": "Unknown biological process"
}